{
  "gene_symbol": "VAMP1",
  "gene": "UniProtKB:P23763",
  "term_id": "GO:0031201",
  "gene_name": "Vesicle-associated membrane protein 1",
  "term_label": "SNARE complex"
}